negative regulation of tatiopterin biosynthetic process [GO:1900975] (BP) Relationships: is a type of negative regulation of biosynthetic process [GO:0009890]; is a type of GO:0010563; is a type of negative regulation of small molecule metabolic process [GO:0062014]; is a type of regulation of tatiopterin biosynthetic process [GO:1900974]; negatively regulates tatiopterin biosynthetic process [GO:1900870] Sources: GOC:TermGenie, GOC:mengo_curators Also known as: down regulation of tatiopterin anabolism, down regulation of tatiopterin biosynthesis, down regulation of tatiopterin biosynthetic process, down regulation of tatiopterin formation, down regulation of tatiopterin synthesis, down-regulation of tatiopterin anabolism, down-regulation of tatiopterin biosynthesis, down-regulation of tatiopterin biosynthetic process, down-regulation of tatiopterin formation, down-regulation of tatiopterin synthesis, downregulation of tatiopterin anabolism, downregulation of tatiopterin biosynthesis, downregulation of tatiopterin biosynthetic process, downregulation of tatiopterin formation, downregulation of tatiopterin synthesis, inhibition of tatiopterin anabolism, inhibition of tatiopterin biosynthesis, inhibition of tatiopterin formation, inhibition of tatiopterin synthesis, negative regulation of tatiopterin anabolism, negative regulation of tatiopterin biosynthesis, negative regulation of tatiopterin formation, negative regulation of tatiopterin synthesis, inhibition of tatiopterin biosynthetic process Definition: Any process that stops, prevents or reduces the frequency, rate or extent of tatiopterin biosynthetic process.